corolla development [GO:0048465] (biological process) Sources: GOC:go_curators Definition: The process whose specific outcome is the progression of the corolla over time, from its formation to the mature structure. Relationships: is a type of floral whorl development [GO:0048438]